{
  "term_id": "GO:0005886",
  "gene_name": "V-type proton ATPase 116 kDa subunit a 4",
  "term_label": "plasma membrane",
  "gene": "UniProtKB:Q9HBG4",
  "gene_symbol": "ATP6V0A4"
}